{
  "term_id": "UNKNOWN:0003",
  "term_label": "Unknown cellular component",
  "gene": "UniProtKB:Q6NVU6",
  "gene_symbol": "UFSP1",
  "gene_name": "Inactive Ufm1-specific protease 1"
}